{
  "term_id": "GO:0030864",
  "term_label": "cortical actin cytoskeleton",
  "gene_symbol": "HIP1",
  "gene_name": "Huntingtin-interacting protein 1",
  "gene": "UniProtKB:O00291"
}